tricyclic triterpenoid biosynthetic process [GO:0010263] (BP) Definition: The chemical reactions and pathways resulting in the formation of tricyclic triterpenoid compounds, terpenoids with 6 isoprene units and 3 carbon rings. Also known as: tricyclic triterpenoid anabolism, tricyclic triterpenoid biosynthesis, tricyclic triterpenoid formation, tricyclic triterpenoid synthesis Relationships: is a type of triterpenoid biosynthetic process [GO:0016104] Sources: GOC:ct